short nephron development [GO:0072030] (biological process) Definition: The process whose specific outcome is the progression of a short nephron over time, from its formation to the mature structure. Short nephrons are associated with mid-cortical and superficial glomeruli, are situated entirely in the outer medulla, and have no thin ascending limb. Subtypes: metanephric short nephron development [GO:0072270] Relationships: is a type of nephron development [GO:0072006] Sources: GOC:mtg_kidney_jan10